{
  "gene_name": "Alpha-crystallin A chain",
  "gene_symbol": "CRYAA",
  "term_id": "GO:0042026",
  "gene": "UniProtKB:P02489",
  "term_label": "protein refolding"
}